positive regulation of asperfuranone biosynthetic process [GO:1900639] (biological process) Definition: Any process that activates or increases the frequency, rate or extent of asperfuranone biosynthetic process. Sources: GOC:TermGenie, GOC:di Also known as: activation of asperfuranone anabolism, activation of asperfuranone biosynthesis, activation of asperfuranone formation, activation of asperfuranone synthesis, positive regulation of asperfuranone anabolism, positive regulation of asperfuranone biosynthesis, positive regulation of asperfuranone formation, positive regulation of asperfuranone synthesis, up regulation of asperfuranone anabolism, up regulation of asperfuranone biosynthesis, up regulation of asperfuranone biosynthetic process, up regulation of asperfuranone formation, up regulation of asperfuranone synthesis, up-regulation of asperfuranone anabolism, up-regulation of asperfuranone biosynthesis, up-regulation of asperfuranone biosynthetic process, up-regulation of asperfuranone formation, up-regulation of asperfuranone synthesis, upregulation of asperfuranone anabolism, upregulation of asperfuranone biosynthesis, upregulation of asperfuranone biosynthetic process, upregulation of asperfuranone formation, upregulation of asperfuranone synthesis, activation of asperfuranone biosynthetic process Relationships: is a type of regulation of asperfuranone biosynthetic process [GO:1900637]; is a type of positive regulation of polyketide biosynthetic process [GO:1900734]; is a type of GO:1902932; positively regulates asperfuranone biosynthetic process [GO:1900554]